{
  "gene_name": "Transcription factor 15",
  "term_label": "regulation of transcription by RNA polymerase II",
  "gene": "UniProtKB:Q12870",
  "gene_symbol": "TCF15",
  "term_id": "GO:0006357"
}